{
  "term_label": "spliceosomal complex",
  "gene_name": "Putative pre-mRNA-splicing factor ATP-dependent RNA helicase DHX32",
  "gene": "UniProtKB:Q7L7V1",
  "term_id": "GO:0005681",
  "gene_symbol": "DHX32"
}